{
  "gene": "UniProtKB:Q9NVS9",
  "term_label": "Unknown cellular component",
  "gene_name": "Pyridoxine-5'-phosphate oxidase",
  "gene_symbol": "PNPO",
  "term_id": "UNKNOWN:0003"
}